{
  "gene": "UniProtKB:Q5VTE6",
  "term_label": "Unknown cellular component",
  "gene_name": "Protein angel homolog 2",
  "gene_symbol": "ANGEL2",
  "term_id": "UNKNOWN:0003"
}